autolysosome [GO:0044754] (cellular component) References: PMID:19008921, PMID:24657946 Sources: GOC:sart, NIF_Subcellular:sao8444068431 Also known as: AVd, degrading autophagic vacuole Definition: A type of secondary lysosome in which a primary lysosome has fused with the outer membrane of an autophagosome or amphisome. It is involved in the second step of autophagy in which it degrades contents with acidic lysosomal hydrolases. Relationships: is a type of secondary lysosome [GO:0005767]